{
  "term_label": "protein folding",
  "gene": "UniProtKB:Q9H3Z4",
  "gene_symbol": "DNAJC5",
  "term_id": "GO:0006457",
  "gene_name": "DnaJ homolog subfamily C member 5"
}